{
  "term_id": "GO:0016604",
  "gene_symbol": "SETX",
  "term_label": "nuclear body",
  "gene": "UniProtKB:Q7Z333",
  "gene_name": "Probable helicase senataxin"
}